hexokinase activity [GO:0004396] (molecular function) Definition: Catalysis of the reaction: ATP + D-hexose = ADP + D-hexose 6-phosphate. Sources: EC:2.7.1.1 Regulation: positively regulated by positive regulation of hexokinase activity [GO:1903301] Subtypes: GO:0004340, D-allose kinase activity [GO:0008787], fructokinase activity [GO:0008865], mannokinase activity [GO:0019158] Also known as: hexokinase type I activity, hexokinase type II activity, hexokinase type III activity, hexokinase type IV (glucokinase) activity, ATP-dependent hexokinase activity, ATP:D-hexose 6-phosphotransferase activity, glucose ATP phosphotransferase activity, hexokinase (phosphorylating), hexokinase D, hexokinase type IV, hexokinase type IV glucokinase activity Relationships: is a type of phosphotransferase activity, alcohol group as acceptor [GO:0016773]; is a type of carbohydrate kinase activity [GO:0019200]